meiotic actomyosin contractile ring [GO:0110086] (cellular component) Definition: A cytoskeletal structure composed of actin filaments, myosin, and myosin-associated proteins that forms beneath the plasma membrane of many cells, including animal cells and yeast cells, in a plane perpendicular to the axis of the meiotic spindle, i.e. the cell division plane. Ring contraction is associated with centripetal growth of the membrane that divides the cytoplasm of the two future daughter cells. In animal cells, the meiotic contractile ring is located inside the plasma membrane at the location of the cleavage furrow. In fungal cells, the meiotic contractile ring forms beneath the plasma membrane of the prospore envelope in preparation for completing cytokinesis. References: PMID:22526418 Sources: GOC:vw Subtypes: prospore contractile ring [GO:0032157] Relationships: is a type of GO:0005826